{
  "gene_symbol": "IFT43",
  "term_id": "GO:0035721",
  "gene_name": "Intraflagellar transport protein 43 homolog",
  "gene": "UniProtKB:Q96FT9",
  "term_label": "intraciliary retrograde transport"
}